4-hydroxyphenylacetate transport [GO:1900754] (biological process) References: PMID:9315705 Sources: GOC:TermGenie Definition: The directed movement of a 4-hydroxyphenylacetate into, out of or within a cell, or between cells, by means of some agent such as a transporter or pore. Also known as: (4-hydroxyphenyl)acetate transport, (p-hydroxyphenyl)acetate transport, 2-(4-hydroxyphenyl)ethanoate transport, 4-hydroxybenzeneacetate transport Relationships: is a type of GO:0015718; is a type of organic hydroxy compound transport [GO:0015850]